{
  "gene": "UniProtKB:Q9BSY4",
  "gene_name": "Coiled-coil-helix-coiled-coil-helix domain-containing protein 5",
  "term_id": "GO:0005758",
  "gene_symbol": "CHCHD5",
  "term_label": "mitochondrial intermembrane space"
}